{
  "gene_symbol": "FAM209B",
  "term_id": "UNKNOWN:0002",
  "gene": "UniProtKB:Q5JX69",
  "gene_name": "Protein FAM209B",
  "term_label": "Unknown biological process"
}